{
  "term_label": "translational elongation",
  "gene": "UniProtKB:P24534",
  "gene_name": "Elongation factor 1-beta",
  "term_id": "GO:0006414",
  "gene_symbol": "EEF1B2"
}